{
  "gene": "UniProtKB:Q9Y2I2",
  "term_id": "GO:0005886",
  "gene_name": "Netrin-G1",
  "gene_symbol": "NTNG1",
  "term_label": "plasma membrane"
}